{
  "gene": "UniProtKB:Q9P272",
  "term_id": "GO:0030488",
  "gene_name": "Probable tRNA methyltransferase 9B",
  "term_label": "tRNA methylation",
  "gene_symbol": "TRMT9B"
}